{
  "term_label": "sensory perception of smell",
  "gene_name": "Olfactory receptor 8D2",
  "term_id": "GO:0007608",
  "gene_symbol": "OR8D2",
  "gene": "UniProtKB:Q9GZM6"
}